{
  "term_label": "RNA methyltransferase activity",
  "gene": "UniProtKB:Q8N3J2",
  "gene_symbol": "METTL4",
  "gene_name": "N(6)-adenine-specific methyltransferase METTL4",
  "term_id": "GO:0008173"
}